regulation of lymphocyte activation [GO:0051249] (biological process) Definition: Any process that modulates the frequency, rate or extent of lymphocyte activation. Subtypes: regulation of natural killer cell activation [GO:0032814], GO:0045619, regulation of lymphocyte proliferation [GO:0050670], GO:0050863, regulation of B cell activation [GO:0050864], negative regulation of lymphocyte activation [GO:0051250], GO:0051251, GO:2000520 Sources: GOC:ai Relationships: is_a regulation of leukocyte activation [GO:0002694]; regulates GO:0046649